{
  "gene_name": "ER degradation-enhancing alpha-mannosidase-like protein 1",
  "gene_symbol": "EDEM1",
  "gene": "UniProtKB:Q92611",
  "term_label": "Unknown molecular function",
  "term_id": "UNKNOWN:0001"
}